{
  "term_label": "chromatin binding",
  "gene_name": "Bifunctional peptidase and arginyl-hydroxylase JMJD5",
  "gene": "UniProtKB:Q8N371",
  "gene_symbol": "KDM8",
  "term_id": "GO:0003682"
}